{
  "term_label": "neurotransmitter receptor activity",
  "term_id": "GO:0030594",
  "gene": "UniProtKB:Q13639",
  "gene_name": "5-hydroxytryptamine receptor 4",
  "gene_symbol": "HTR4"
}